{
  "gene_name": "Pro-opiomelanocortin",
  "term_label": "G protein-coupled receptor binding",
  "gene": "UniProtKB:P01189",
  "term_id": "GO:0001664",
  "gene_symbol": "POMC"
}